negative regulation of CD4-positive, alpha-beta T cell costimulation [GO:1900280] (biological process) Definition: Any process that stops, prevents or reduces the frequency, rate or extent of CD4-positive, alpha-beta T cell costimulation. Sources: GOC:BHF, GOC:TermGenie, GOC:pr Also known as: down regulation of CD4-positive, alpha beta T cell costimulation, down-regulation of CD4-positive, alpha beta T cell costimulation, downregulation of CD4-positive, alpha beta T cell costimulation, negative regulation of CD4-positive, alpha beta T cell costimulation, inhibition of CD4-positive, alpha beta T cell costimulation Relationships: is a type of regulation of CD4-positive, alpha-beta T cell costimulation [GO:1900279]; is a type of GO:2000524; negatively regulates GO:0035783